{
  "gene_symbol": "FOXP4",
  "term_label": "DNA-binding transcription repressor activity, RNA polymerase II-specific",
  "term_id": "GO:0001227",
  "gene": "UniProtKB:Q8IVH2",
  "gene_name": "Forkhead box protein P4"
}